{
  "term_id": "GO:0031012",
  "gene_symbol": "ADAMTS3",
  "gene_name": "A disintegrin and metalloproteinase with thrombospondin motifs 3",
  "term_label": "extracellular matrix",
  "gene": "UniProtKB:O15072"
}